{
  "gene_name": "Claudin-1",
  "gene": "UniProtKB:O95832",
  "gene_symbol": "CLDN1",
  "term_label": "plasma membrane",
  "term_id": "GO:0005886"
}